{
  "term_id": "UNKNOWN:0002",
  "gene": "UniProtKB:Q92737",
  "term_label": "Unknown biological process",
  "gene_name": "Ras-like protein family member 10A",
  "gene_symbol": "RASL10A"
}